response to mitotic DNA replication checkpoint signaling [GO:0072444] (biological process) Definition: A process that occurs in response to signals generated as a result of mitotic DNA replication checkpoint signaling. Sources: GOC:mtg_cell_cycle Also known as: S-M checkpoint effector process, mitotic DNA replication checkpoint effector process, response to S-M checkpoint signaling, response to signal involved in S-M checkpoint, response to signal involved in mitotic DNA replication checkpoint Relationships: is a type of GO:0072414; is_a response to DNA replication checkpoint signaling [GO:0072438]